{
  "term_label": "centriole",
  "gene": "UniProtKB:Q9P2P6",
  "gene_symbol": "STARD9",
  "term_id": "GO:0005814",
  "gene_name": "StAR-related lipid transfer protein 9"
}